peptidoglycan recognition protein signaling pathway [GO:0061057] (BP) References: PMID:18688280, PMID:24706930 Sources: GOC:dph Definition: The series of molecular signals initiated by binding of peptidoglycan to a receptor and ending with regulation of a downstream cellular process. The main outcome of the Imd signaling is the production of antimicrobial peptides. Regulation: RO_0002211 by regulation of peptidoglycan recognition protein signaling pathway [GO:0061058]; RO_0002213 by positive regulation of peptidoglycan recognition protein signaling pathway [GO:0061059]; negatively regulated by negative regulation of peptidoglycan recognition protein signaling pathway [GO:0061060] Relationships: is a type of GO:0002221; is part of GO:0042742 Also known as: Imd signaling pathway, Imd signalling pathway, PGRP signaling pathway, immune deficiency pathway, immune deficiency signaling pathway